{
  "term_id": "GO:0006788",
  "gene_symbol": "HMOX1",
  "gene_name": "Heme oxygenase 1",
  "term_label": "heme oxidation",
  "gene": "UniProtKB:P09601"
}